{
  "gene_symbol": "BMP7",
  "term_id": "GO:0030509",
  "term_label": "BMP signaling pathway",
  "gene": "UniProtKB:P18075",
  "gene_name": "Bone morphogenetic protein 7"
}